{
  "term_id": "GO:0004984",
  "gene_name": "Olfactory receptor 6V1",
  "gene_symbol": "OR6V1",
  "gene": "UniProtKB:Q8N148",
  "term_label": "olfactory receptor activity"
}